trimming of terminal mannose on C branch [GO:0036510] (biological process) Relationships: is a type of GO:1904380 References: PMID:20065073 Sources: GOC:PARL, GOC:bf Note: Consider also annotating to 'mannosyl-oligosaccharide 1,2-alpha-mannosidase activity ; GO:0004571'. Definition: The removal of an alpha-1,2-linked mannose from the C-chain of a glycoprotein oligosaccharide in the endoplasmic reticulum. Also known as: glycoprotein mannose trimming on C branch, conversion of (Man)9(GlcNAc)2 to (Man)8C(GlcNAc)2, conversion of M9 to M8C